{
  "gene": "UniProtKB:P43686",
  "term_id": "GO:0008540",
  "gene_symbol": "PSMC4",
  "gene_name": "26S proteasome regulatory subunit 6B",
  "term_label": "proteasome regulatory particle, base subcomplex"
}